{
  "gene_name": "Gamma-tubulin complex component 2",
  "gene_symbol": "TUBGCP2",
  "term_id": "GO:0051225",
  "gene": "UniProtKB:Q9BSJ2",
  "term_label": "spindle assembly"
}